{
  "gene_name": "Probable non-functional immunoglobulin lambda variable 5-48",
  "gene_symbol": "IGLV5-48",
  "term_label": "immunoglobulin complex",
  "gene": "UniProtKB:A0A075B6I7",
  "term_id": "GO:0019814"
}